{
  "term_label": "cellular response to oxidative stress",
  "term_id": "GO:0034599",
  "gene": "UniProtKB:Q16236",
  "gene_name": "Nuclear factor erythroid 2-related factor 2",
  "gene_symbol": "NFE2L2"
}